{
  "gene": "UniProtKB:Q9ULV5",
  "term_label": "RNA polymerase II cis-regulatory region sequence-specific DNA binding",
  "term_id": "GO:0000978",
  "gene_name": "Heat shock factor protein 4",
  "gene_symbol": "HSF4"
}